{
  "gene": "UniProtKB:Q8IZJ1",
  "term_label": "netrin receptor activity",
  "gene_name": "Netrin receptor UNC5B",
  "gene_symbol": "UNC5B",
  "term_id": "GO:0005042"
}